establishment or maintenance of neuroblast polarity [GO:0045196] (biological process) Subtypes: GO:0045200, maintenance of neuroblast polarity [GO:0045201] Also known as: establishment and/or maintenance of neuroblast cell polarity Regulation: negatively regulated by negative regulation of establishment or maintenance of neuroblast polarity [GO:2000248] Relationships: is_a establishment or maintenance of cell polarity [GO:0007163]; is part of asymmetric neuroblast division [GO:0055059] Definition: Any cellular process that results in the specification, formation or maintenance of the apicobasal polarity of a neuroblast cell, a progenitor of the central nervous system. References: PMID:19375318, PMID:20066083 Sources: GOC:bf, GOC:mah, GOC:mtg_sensu